deUFMylase activity [GO:0071567] (molecular function) References: PMID:17182609, PMID:20018847 Sources: GOC:sp Relationships: is a type of cysteine-type peptidase activity [GO:0008234]; is a type of ubiquitin-like protein peptidase activity [GO:0019783] Also known as: UFM1 hydrolase activity Definition: A thiol-dependent isopeptidase activity that cleaves UFM1 from a target protein to which it is conjugated.